{
  "term_label": "Unknown biological process",
  "gene_name": "Olfactory receptor 4S2",
  "gene_symbol": "OR4S2",
  "gene": "UniProtKB:Q8NH73",
  "term_id": "UNKNOWN:0002"
}